{
  "gene_name": "Inner nuclear membrane protein Man1",
  "gene_symbol": "LEMD3",
  "term_label": "Unknown cellular component",
  "term_id": "UNKNOWN:0003",
  "gene": "UniProtKB:Q9Y2U8"
}